{
  "gene_name": "Humanin-like 3",
  "term_label": "Unknown cellular component",
  "gene": "UniProtKB:P0CJ70",
  "term_id": "UNKNOWN:0003",
  "gene_symbol": "MTRNR2L3"
}